{
  "term_id": "GO:0005783",
  "gene_symbol": "RHBDD1",
  "gene": "UniProtKB:Q8TEB9",
  "term_label": "endoplasmic reticulum",
  "gene_name": "Rhomboid-related protein 4"
}